{
  "gene_symbol": "SHC3",
  "gene_name": "SHC-transforming protein 3",
  "term_label": "plasma membrane",
  "term_id": "GO:0005886",
  "gene": "UniProtKB:Q92529"
}